{
  "gene_symbol": "FAM177B",
  "gene_name": "Protein FAM177B",
  "term_id": "UNKNOWN:0001",
  "gene": "UniProtKB:A6PVY3",
  "term_label": "Unknown molecular function"
}